leukotriene B4 biosynthetic process [GO:0097251] (biological process) Sources: GOC:yaf Also known as: LTB4 anabolism, LTB4 biosynthesis, LTB4 formation, LTB4 synthesis, leukotriene B4 anabolism, leukotriene B4 biosynthesis, leukotriene B4 formation, leukotriene B4 synthesis Definition: The chemical reactions and pathways resulting in the formation of leukotriene B4, a leukotriene composed of (6Z,8E,10E,14Z)-eicosatetraenoic acid having (5S)- and (12R)-hydroxy substituents. Relationships: is_a leukotriene biosynthetic process [GO:0019370]; is a type of leukotriene B4 metabolic process [GO:0036102]; is a type of long-chain fatty acid biosynthetic process [GO:0042759]; is a type of fatty acid derivative biosynthetic process [GO:1901570]